ganglioside GM1 transport to membrane [GO:1905572] (biological process) Definition: The directed movement of ganglioside GM1 to membrane. References: PMID:1454804 Sources: GOC:TermGenie, GO_REF:0000078 Relationships: is a type of ceramide transport [GO:0035627]; is a type of glycolipid transport [GO:0046836]; is a type of GO:0046942; is a type of localization within membrane [GO:0051668]